{
  "gene_symbol": "EFTUD2",
  "term_label": "U2-type catalytic step 2 spliceosome",
  "gene": "UniProtKB:Q15029",
  "gene_name": "116 kDa U5 small nuclear ribonucleoprotein component",
  "term_id": "GO:0071007"
}